{
  "term_label": "serine-type endopeptidase activity",
  "term_id": "GO:0004252",
  "gene": "UniProtKB:P10144",
  "gene_name": "Granzyme B",
  "gene_symbol": "GZMB"
}